{
  "gene_symbol": "RINT1",
  "gene": "UniProtKB:Q6NUQ1",
  "term_label": "Dsl1/NZR complex",
  "gene_name": "RAD50-interacting protein 1",
  "term_id": "GO:0070939"
}